{
  "gene": "UniProtKB:A0A087WUM9",
  "gene_name": "Uncharacterized protein",
  "term_label": "Unknown cellular component",
  "term_id": "UNKNOWN:0003",
  "gene_symbol": "A0A087WUM9"
}